{
  "term_label": "Unknown cellular component",
  "gene_name": "Mitochondrial 10-formyltetrahydrofolate dehydrogenase",
  "gene": "UniProtKB:Q3SY69",
  "term_id": "UNKNOWN:0003",
  "gene_symbol": "ALDH1L2"
}